{
  "gene_symbol": "NMUR2",
  "gene": "UniProtKB:Q9GZQ4",
  "term_label": "neuropeptide receptor activity",
  "term_id": "GO:0008188",
  "gene_name": "Neuromedin-U receptor 2"
}